{
  "gene": "UniProtKB:Q9H9Z2",
  "term_id": "GO:0005634",
  "gene_symbol": "LIN28A",
  "term_label": "nucleus",
  "gene_name": "Protein lin-28 homolog A"
}